lipoamide binding [GO:0043544] (molecular function) Relationships: is a type of amide binding [GO:0033218]; is a type of sulfur compound binding [GO:1901681] Definition: Binding to lipoamide, the functional form of lipoic acid in which the carboxyl group is attached to protein by an amide linkage to a lysine amino group. Sources: GOC:go_curators